{
  "term_id": "GO:0008143",
  "gene_symbol": "KHDRBS1",
  "gene": "UniProtKB:Q07666",
  "term_label": "poly(A) binding",
  "gene_name": "KH domain-containing, RNA-binding, signal transduction-associated protein 1"
}